{
  "gene": "UniProtKB:A8MT69",
  "gene_name": "Centromere protein X",
  "term_label": "resolution of meiotic recombination intermediates",
  "term_id": "GO:0000712",
  "gene_symbol": "CENPX"
}